P-type transmembrane transporter activity [GO:0140358] (molecular function) Definition: Primary active transporter that auto-phosphorylates (hence P) at a key conserved aspartate residue, generating a conformational change that allows transport of the substrate. Hydrolysis of the phosphorylated Asp residue, catalyzed by the actuator (A) domain, results in another state with occluded substrates. Upon dissociation of Mg2+ and Pi, the enzyme reverts to the initial state, in which the counter-transported substrate is released into the cytosol. References: PMID:18075584, PMID:25918123 Also known as: E1-E2 ATPase, P-type ATPase Relationships: is a type of ATPase-coupled transmembrane transporter activity [GO:0042626] Subtypes: P-type ion transporter activity [GO:0015662]